plus-end-directed microtubule motor activity [GO:0008574] (molecular function) Relationships: is a type of GO:0003777 Definition: A motor activity that generates movement along a microtubule toward the plus end, driven by ATP hydrolysis. References: PMID:32842864 Sources: GOC:vw Also known as: ATP-dependent microtubule motor activity, plus-end-directed, ATP-dependent plus-end-directed microtubule motor activity, microtubule motor activity, plus-end-directed, plus-end-directed ATP-dependent microtubule motor activity, kinesin ATP phosphohydrolase (plus-end-directed), plus-end-directed kinesin ATPase activity, kinesin activity